{
  "gene": "UniProtKB:Q8N0W7",
  "term_label": "Unknown cellular component",
  "gene_name": "FMR1 neighbor protein",
  "term_id": "UNKNOWN:0003",
  "gene_symbol": "FMR1NB"
}